superior olivary nucleus morphogenesis [GO:0021719] (BP) Definition: The process in which the anatomical structure of the superior olivary nucleus is generated and organized. In mice, the superior olivary nucleus is a small cylindrical mass on the dorsal surface of the lateral part of the trapezoid body of the pons, and it is situated immediately above the inferior olivary nucleus. It receives projections from the cochlear nucleus and thus is involved in the perception of sound. Relationships: is a type of anatomical structure morphogenesis [GO:0009653]; is part of GO:0021583; is part of superior olivary nucleus development [GO:0021718] Sources: GOC:cls, GOC:dgh, GOC:dph, GOC:jid, GO_REF:0000021 Also known as: superior olive morphogenesis